{
  "gene_symbol": "STIMATE",
  "term_label": "Unknown biological process",
  "term_id": "UNKNOWN:0002",
  "gene": "UniProtKB:Q86TL2",
  "gene_name": "Store-operated calcium entry regulator STIMATE"
}